peptide lactyltransferase (ATP-dependent) activity [GO:0141207] (molecular function) Definition: Catalysis of the reaction: lactate + ATP + L-lysyl-[protein] = N(6)-lactoyl-L-lysyl-[protein]+ AMP + diphosphate. Can also act on free lactate. Relationships: is a type of ligase activity, forming phosphoric ester bonds [GO:0016886]; is a type of GO:0140096 Also known as: peptide lactyltransferase activity, peptide lactyltransferase (ATP dependent) activity References: PMID:38512451, PMID:38653238 Sources: RHEA:80271